{
  "gene_name": "Putative exonuclease GOR",
  "gene": "UniProtKB:Q8IX06",
  "term_id": "GO:0031125",
  "gene_symbol": "REXO1L1P",
  "term_label": "rRNA 3'-end processing"
}